peroxisome inheritance [GO:0045033] (biological process) Note: Note that 'vectorial' is used in the definition in the mathematical and physical sense of pertaining to 'a quantity having direction as well as magnitude, especially as determining the position of one point in space relative to another. Definition: The acquisition of peroxisomes by daughter cells from the mother cell after replication. In Saccharomyces cerevisiae, the number of peroxisomes cells is fairly constant; a subset of the organelles are targeted and segregated to the bud in a highly ordered, vectorial process. Efficient segregation of peroxisomes from mother to bud is dependent on the actin cytoskeleton, and active movement of peroxisomes along actin filaments is driven by the class V myosin motor protein, Myo2p. References: PMID:11733545 Relationships: is a type of peroxisome organization [GO:0007031]; is a type of organelle inheritance [GO:0048308]